{
  "gene_symbol": "RASA4B",
  "gene_name": "Ras GTPase-activating protein 4B",
  "term_id": "GO:1902531",
  "term_label": "regulation of intracellular signal transduction",
  "gene": "UniProtKB:C9J798"
}